{
  "term_id": "GO:0005634",
  "gene_symbol": "OLIG1",
  "gene": "UniProtKB:Q8TAK6",
  "term_label": "nucleus",
  "gene_name": "Oligodendrocyte transcription factor 1"
}